circadian regulation of heart rate [GO:0003053] (biological process) Subtypes: GO:0003055 Relationships: is a type of regulation of heart rate [GO:0002027]; is a type of circadian rhythm [GO:0007623]; is_a multicellular organismal process [GO:0032501] Definition: Any process in which an organism modulates its heart rate at different values with a regularity of approximately 24 hours. Sources: GOC:mtg_cardio, GOC:rl Also known as: circadian regulation of heart contraction rate